{
  "gene": "UniProtKB:Q7Z3D4",
  "term_label": "Golgi organization",
  "gene_name": "LysM and putative peptidoglycan-binding domain-containing protein 3",
  "gene_symbol": "LYSMD3",
  "term_id": "GO:0007030"
}